{
  "term_id": "GO:0009986",
  "gene": "UniProtKB:Q8WTV0",
  "gene_name": "Scavenger receptor class B member 1",
  "gene_symbol": "SCARB1",
  "term_label": "cell surface"
}